{
  "gene": "UniProtKB:Q9H3R2",
  "term_id": "UNKNOWN:0001",
  "term_label": "Unknown molecular function",
  "gene_symbol": "MUC13",
  "gene_name": "Mucin-13"
}